{
  "gene_symbol": "ZNF648",
  "gene_name": "Zinc finger protein 648",
  "term_label": "regulation of DNA-templated transcription",
  "term_id": "GO:0006355",
  "gene": "UniProtKB:Q5T619"
}